positive regulation of hair cycle [GO:0042635] (biological process) Definition: Any process that activates or increases the frequency, rate or extent of the cyclical phases of growth (anagen), regression (catagen), quiescence (telogen), and shedding (exogen) in the life of a hair. Relationships: is a type of GO:0042634; is a type of positive regulation of multicellular organismal process [GO:0051240]; positively regulates hair cycle [GO:0042633] References: PMID:12230507 Sources: GOC:go_curators Also known as: up regulation of hair cycle, up-regulation of hair cycle, upregulation of hair cycle, activation of hair cycle, stimulation of hair cycle